{
  "gene_name": "Proprotein convertase subtilisin_kexin type 6",
  "gene_symbol": "PCSK6",
  "term_label": "cell surface",
  "term_id": "GO:0009986",
  "gene": "UniProtKB:P29122"
}